{
  "term_label": "Rho protein signal transduction",
  "gene_symbol": "GNA12",
  "gene": "UniProtKB:Q03113",
  "term_id": "GO:0007266",
  "gene_name": "Guanine nucleotide-binding protein subunit alpha-12"
}